{
  "term_id": "UNKNOWN:0001",
  "gene_symbol": "LOC100996750",
  "gene": "UniProtKB:A0A140TA64",
  "term_label": "Unknown molecular function",
  "gene_name": "Uncharacterized protein"
}